muscle tendon junction [GO:0005927] (cellular component) Definition: A cell-substrate junction found at the terminal anchorage site of skeletal muscle cells to tendons. References: PMID:12842007 Sources: GOC:mtg_muscle Relationships: is a type of cell-substrate junction [GO:0030055] Also known as: myotendinous junction